regulation of bone mineralization involved in bone maturation [GO:1900157] (biological process) Definition: Any process that modulates the frequency, rate or extent of bone mineralization involved in bone maturation. Sources: GOC:BHF, GOC:TermGenie Relationships: is a type of regulation of bone mineralization [GO:0030500]; regulates bone mineralization involved in bone maturation [GO:0035630] Subtypes: negative regulation of bone mineralization involved in bone maturation [GO:1900158], positive regulation of bone mineralization involved in bone maturation [GO:1900159]